detection of parasitic plant [GO:0002243] (biological process) Definition: The series of events in which a stimulus from a parasitic plant is received and converted into a molecular signal. References: PMID:16547862 Sources: GOC:add Relationships: is a type of response to parasitic plant [GO:0002241]; is a type of detection of symbiont [GO:0009602]